{
  "gene": "UniProtKB:A6NC98",
  "term_label": "cytoplasmic microtubule organization",
  "gene_symbol": "CCDC88B",
  "gene_name": "Coiled-coil domain-containing protein 88B",
  "term_id": "GO:0031122"
}